{
  "gene": "UniProtKB:Q15822",
  "term_id": "GO:0007271",
  "gene_name": "Neuronal acetylcholine receptor subunit alpha-2",
  "term_label": "synaptic transmission, cholinergic",
  "gene_symbol": "CHRNA2"
}